ABC-type xenobiotic transporter activity [GO:0008559] (molecular function) Relationships: is a type of GO:0042910; is a type of GO:0140359 Definition: Catalysis of the reaction: ATP + H2O + xenobiotic(in) = ADP + phosphate + xenobiotic(out). Subtypes: ABC-type bacteriocin transporter activity [GO:0043214] Also known as: ATP-dependent xenobiotic transmembrane transporter activity, xenobiotic transmembrane transporting ATPase activity, xenobiotic ABC transporter, ATP phosphohydrolase (xenobiotic-exporting), ATPase-coupled xenobiotic transmembrane transporter activity, MDR protein, P-glycoprotein, PDR protein, multidrug resistance exporter, multidrug-resistance protein, pleiotropic-drug-resistance protein Sources: EC:7.6.2.2